{
  "gene_symbol": "EFHC1",
  "term_id": "GO:0072686",
  "gene": "UniProtKB:Q5JVL4",
  "gene_name": "EF-hand domain-containing protein 1",
  "term_label": "mitotic spindle"
}